pyochelin catabolic process [GO:0042865] (biological process) Also known as: pyochelin breakdown, pyochelin catabolism, pyochelin degradation Relationships: is a type of phenol-containing compound catabolic process [GO:0019336]; is a type of sulfur compound catabolic process [GO:0044273]; is a type of siderophore catabolic process [GO:0046215]; is a type of carboxylic acid catabolic process [GO:0046395] Definition: The chemical reactions and pathways resulting in the breakdown of the siderochrome pyochelin (2-(2-o-hydroxyphenyl-2-thiazolin-4-yl)-3-methylthiazolidine-4-carboxylic acid). References: PMID:6794030 Sources: GOC:jl